{
  "gene": "UniProtKB:Q96MR9",
  "gene_symbol": "ZNF560",
  "term_label": "RNA polymerase II transcription regulatory region sequence-specific DNA binding",
  "gene_name": "Zinc finger protein 560",
  "term_id": "GO:0000977"
}